{
  "gene": "UniProtKB:H3BQW9",
  "term_id": "UNKNOWN:0001",
  "gene_name": "Protein FAM229A",
  "gene_symbol": "FAM229A",
  "term_label": "Unknown molecular function"
}